{
  "gene_name": "E3 ubiquitin-protein ligase ZNRF4",
  "term_id": "GO:0061630",
  "gene_symbol": "ZNRF4",
  "gene": "UniProtKB:Q8WWF5",
  "term_label": "ubiquitin protein ligase activity"
}